deoxyribonuclease I activity [GO:0004530] (molecular function) Definition: Catalysis of the endonucleolytic cleavage of DNA to 5'-phosphodinucleotide and 5'-phosphooligonucleotide end products. Sources: EC:3.1.21.1 Also known as: DNase activity, deoxyribonuclease (pancreatic), pancreatic DNase activity, pancreatic deoxyribonuclease, pancreatic dornase, thymonuclease activity, DNA depolymerase activity, DNA endonuclease activity, DNA nuclease activity, DNAase activity, DNase I, Escherichia coli endonuclease I, alkaline DNase activity, alkaline deoxyribonuclease activity, deoxyribonuclease A, deoxyribonucleic phosphatase activity, dornava, dornavac, endodeoxyribonuclease I, thymonuclease, dornase activity Relationships: is a type of DNA endonuclease activity, producing 5'-phosphomonoesters [GO:0016888]